{
  "term_id": "GO:0032332",
  "gene_symbol": "GDF5",
  "gene": "UniProtKB:P43026",
  "gene_name": "Growth_differentiation factor 5",
  "term_label": "positive regulation of chondrocyte differentiation"
}